hydrolase activity, acting on acid anhydrides [GO:0016817] (molecular function) Sources: GOC:jl Also known as: hydrolase activity, acting on acid anhydrides, involved in cellular and subcellular movement Relationships: is a type of hydrolase activity [GO:0016787] Definition: Catalysis of the hydrolysis of any acid anhydride. Subtypes: hydrolase activity, acting on acid anhydrides, in phosphorus-containing anhydrides [GO:0016818], hydrolase activity, acting on acid anhydrides, in sulfonyl-containing anhydrides [GO:0016819]